{
  "term_id": "GO:0050911",
  "gene_name": "Putative olfactory receptor 2W5 pseudogene",
  "gene": "UniProtKB:A6NFC9",
  "gene_symbol": "OR2W5P",
  "term_label": "detection of chemical stimulus involved in sensory perception of smell"
}